pheromone catabolic process [GO:0042812] (biological process) Relationships: is a type of GO:0042447; is a type of pheromone metabolic process [GO:0042810] Sources: ISBN:0198506732 Definition: The chemical reactions and pathways resulting in the breakdown of pheromones, a substance that is secreted and released by an organism and detected by a second organism of the same or a closely related species, in which it causes a specific reaction, such as a definite behavioral reaction or a developmental process. Also known as: pheromone breakdown, pheromone catabolism, pheromone degradation